{
  "term_label": "cyclic-GMP-AMP transmembrane import across plasma membrane",
  "gene": "UniProtKB:Q6NSJ5",
  "term_id": "GO:0140361",
  "gene_symbol": "LRRC8E",
  "gene_name": "Volume-regulated anion channel subunit LRRC8E"
}